{
  "gene_symbol": "AVEN",
  "term_label": "Unknown molecular function",
  "term_id": "UNKNOWN:0001",
  "gene": "UniProtKB:Q9NQS1",
  "gene_name": "Cell death regulator Aven"
}